{
  "gene_symbol": "ARHGEF11",
  "term_label": "G protein-coupled receptor signaling pathway",
  "term_id": "GO:0007186",
  "gene": "UniProtKB:O15085",
  "gene_name": "Rho guanine nucleotide exchange factor 11"
}